{
  "term_label": "endoplasmic reticulum membrane",
  "term_id": "GO:0005789",
  "gene_symbol": "LMAN1",
  "gene_name": "Protein ERGIC-53",
  "gene": "UniProtKB:P49257"
}